{
  "gene_name": "Actin-like protein 8",
  "term_id": "GO:0007409",
  "gene_symbol": "ACTL8",
  "gene": "UniProtKB:Q9H568",
  "term_label": "axonogenesis"
}